{
  "gene_name": "Medium-wave-sensitive opsin 1",
  "term_id": "GO:0007602",
  "gene_symbol": "OPN1MW",
  "gene": "UniProtKB:P04001",
  "term_label": "phototransduction"
}